{
  "gene": "UniProtKB:P46782",
  "gene_name": "Small ribosomal subunit protein uS7",
  "gene_symbol": "RPS5",
  "term_label": "mRNA binding",
  "term_id": "GO:0003729"
}